{
  "gene_name": "RNA-binding protein 26",
  "term_label": "Unknown biological process",
  "term_id": "UNKNOWN:0002",
  "gene_symbol": "RBM26",
  "gene": "UniProtKB:Q5T8P6"
}